{
  "term_id": "GO:0005886",
  "term_label": "plasma membrane",
  "gene": "UniProtKB:Q9NT99",
  "gene_name": "Leucine-rich repeat-containing protein 4B",
  "gene_symbol": "LRRC4B"
}